ecdysone oxidase activity [GO:0047875] (molecular function) Definition: Catalysis of the reaction: Ecdysone + O2 = 3-dehydroecdysone + H2O2. Also known as: beta-ecdysone oxidase activity, ecdysone:oxygen 3-oxidoreductase activity Relationships: is_a oxidoreductase activity, acting on the CH-OH group of donors, oxygen as acceptor [GO:0016899] Sources: EC:1.1.3.16, RHEA:11796